{
  "gene": "UniProtKB:Q96LS8",
  "term_label": "Unknown biological process",
  "gene_symbol": "C2orf48",
  "term_id": "UNKNOWN:0002",
  "gene_name": "Putative uncharacterized protein C2orf48"
}